{
  "gene_name": "CD302 antigen",
  "term_id": "UNKNOWN:0001",
  "gene": "UniProtKB:Q8IX05",
  "term_label": "Unknown molecular function",
  "gene_symbol": "CD302"
}